{
  "gene": "UniProtKB:Q13825",
  "term_label": "enoyl-CoA hydratase activity",
  "term_id": "GO:0004300",
  "gene_symbol": "AUH",
  "gene_name": "Methylglutaconyl-CoA hydratase, mitochondrial"
}